{
  "term_label": "medium-chain fatty acid-CoA ligase activity",
  "gene": "UniProtKB:Q96CM8",
  "gene_name": "Medium-chain acyl-CoA ligase ACSF2, mitochondrial",
  "term_id": "GO:0031956",
  "gene_symbol": "ACSF2"
}